{
  "gene": "UniProtKB:P06737",
  "term_id": "GO:0005980",
  "term_label": "glycogen catabolic process",
  "gene_symbol": "PYGL",
  "gene_name": "Glycogen phosphorylase, liver form"
}